{
  "term_label": "immunoglobulin mediated immune response",
  "term_id": "GO:0016064",
  "gene_name": "Immunoglobulin heavy variable 3-53",
  "gene": "UniProtKB:P01767",
  "gene_symbol": "IGHV3-53"
}